{
  "gene_name": "Putative protein phosphatase inhibitor 2-like protein 1",
  "gene_symbol": "PPP1R2P1",
  "term_label": "Unknown cellular component",
  "gene": "UniProtKB:Q96PQ5",
  "term_id": "UNKNOWN:0003"
}